medial cortex septin ring [GO:0036391] (cellular component) Definition: A ring-shaped structure that forms at the medial cortex of a symmetrically dividing cell at the onset of cytokinesis; composed of members of the conserved family of filament forming proteins called septins as well as septin-associated proteins. Relationships: is a type of septin ring [GO:0005940]; is a type of cleavage apparatus septin structure [GO:0032161]; is part of medial cortex [GO:0031097] References: PMID:16009555 Sources: GOC:vw